{
  "gene_symbol": "NELFA",
  "gene": "UniProtKB:Q9H3P2",
  "term_label": "molecular adaptor activity",
  "term_id": "GO:0060090",
  "gene_name": "Negative elongation factor A"
}